{
  "term_label": "phosphatidylcholine metabolic process",
  "term_id": "GO:0046470",
  "gene_name": "Otoconin-90",
  "gene": "UniProtKB:Q02509",
  "gene_symbol": "OC90"
}